{
  "gene_symbol": "ACYP2",
  "gene_name": "Acylphosphatase-2",
  "term_id": "GO:0003998",
  "gene": "UniProtKB:P14621",
  "term_label": "acylphosphatase activity"
}